{
  "gene_symbol": "SRI",
  "term_id": "UNKNOWN:0003",
  "gene": "UniProtKB:P30626",
  "gene_name": "Sorcin",
  "term_label": "Unknown cellular component"
}